{
  "gene": "UniProtKB:P15382",
  "term_id": "GO:0086011",
  "gene_symbol": "KCNE1",
  "gene_name": "Potassium voltage-gated channel subfamily E member 1",
  "term_label": "membrane repolarization during action potential"
}